{
  "term_id": "GO:0005886",
  "term_label": "plasma membrane",
  "gene_name": "ATP-binding cassette sub-family C member 6",
  "gene_symbol": "ABCC6",
  "gene": "UniProtKB:O95255"
}